histone deacetylase complex [GO:0000118] (cellular component) Relationships: is a type of nuclear protein-containing complex [GO:0140513]; is a type of GO:1902494; is part of nucleoplasm [GO:0005654] Note: Note that this term represents a location, not a function; the activity possessed by this complex is mentioned in the definition for the purpose of describing and distinguishing the complex. The function of this complex is represented by the molecular function term 'histone deacetylase activity ; GO:0004407'. Also known as: HDAC complex Definition: A protein complex that possesses histone deacetylase activity. Sources: GOC:mah Subtypes: Swr1 complex [GO:0000812], NuRD complex [GO:0016581], Set3 complex [GO:0034967], Rpd3L-Expanded complex [GO:0070210], Snt2C complex [GO:0070211], Sin3-type complex [GO:0070822], HDA1 complex [GO:0070823]